{
  "gene_symbol": "H1-9P",
  "gene_name": "Putative spermatid-specific linker histone H1-like protein",
  "gene": "UniProtKB:P60008",
  "term_label": "double-stranded DNA binding",
  "term_id": "GO:0003690"
}